{
  "term_label": "histone H3K9 methyltransferase activity",
  "term_id": "GO:0046974",
  "gene_name": "Histone-lysine N-methyltransferase SETDB1",
  "gene_symbol": "SETDB1",
  "gene": "UniProtKB:Q15047"
}